{
  "term_label": "neuron projection",
  "gene_symbol": "CHRNE",
  "term_id": "GO:0043005",
  "gene": "UniProtKB:Q04844",
  "gene_name": "Acetylcholine receptor subunit epsilon"
}